{
  "gene_symbol": "TCAIM",
  "term_label": "Unknown molecular function",
  "gene": "UniProtKB:Q8N3R3",
  "term_id": "UNKNOWN:0001",
  "gene_name": "T-cell activation inhibitor, mitochondrial"
}